{
  "term_id": "GO:0042391",
  "gene": "UniProtKB:A5X5Y0",
  "term_label": "regulation of membrane potential",
  "gene_name": "5-hydroxytryptamine receptor 3E",
  "gene_symbol": "HTR3E"
}